{
  "gene_name": "Amphiphysin",
  "term_id": "GO:0008021",
  "gene": "UniProtKB:P49418",
  "term_label": "synaptic vesicle",
  "gene_symbol": "AMPH"
}